{
  "term_id": "GO:0000981",
  "gene_symbol": "FOXB2",
  "gene": "UniProtKB:Q5VYV0",
  "term_label": "DNA-binding transcription factor activity, RNA polymerase II-specific",
  "gene_name": "Forkhead box protein B2"
}